{
  "term_id": "GO:0038043",
  "term_label": "interleukin-5-mediated signaling pathway",
  "gene": "UniProtKB:P32927",
  "gene_symbol": "CSF2RB",
  "gene_name": "Cytokine receptor common subunit beta"
}